response to biotic stimulus [GO:0009607] (biological process) Definition: Any process that results in a change in state or activity of a cell or an organism (in terms of movement, secretion, enzyme production, gene expression, etc.) as a result of a biotic stimulus, a stimulus caused or produced by a living organism. Note: Note that this term is in the subset of terms that should not be used for direct gene product annotation. Instead, select a child term or, if no appropriate child term exists, please request a new term. Direct annotations to this term may be amended during annotation QC. Sources: GOC:hb Relationships: is a type of response to stimulus [GO:0050896] Also known as: response to biotic stress Regulation: regulated by regulation of response to biotic stimulus [GO:0002831]; negatively regulated by GO:0002832; positively regulated by positive regulation of response to biotic stimulus [GO:0002833] Subtypes: response to tumor cell [GO:0002347], detection of biotic stimulus [GO:0009595], GO:0036180, response to external biotic stimulus [GO:0043207], cellular response to biotic stimulus [GO:0071216], response to lectin [GO:1990840]